{
  "term_label": "extracellular space",
  "gene_symbol": "GZMB",
  "gene_name": "Granzyme B",
  "gene": "UniProtKB:P10144",
  "term_id": "GO:0005615"
}